{
  "gene_name": "Fatty acid-binding protein 5",
  "term_label": "fatty acid transport",
  "gene": "UniProtKB:Q01469",
  "gene_symbol": "FABP5",
  "term_id": "GO:0015908"
}